{
  "gene": "UniProtKB:P14867",
  "term_label": "synaptic transmission, GABAergic",
  "term_id": "GO:0051932",
  "gene_name": "Gamma-aminobutyric acid receptor subunit alpha-1",
  "gene_symbol": "GABRA1"
}